{
  "gene_symbol": "KRTAP25-1",
  "term_id": "UNKNOWN:0003",
  "gene_name": "Keratin-associated protein 25-1",
  "gene": "UniProtKB:Q3LHN0",
  "term_label": "Unknown cellular component"
}